{
  "term_id": "GO:0006887",
  "term_label": "exocytosis",
  "gene": "UniProtKB:Q12846",
  "gene_symbol": "STX4",
  "gene_name": "Syntaxin-4"
}